{
  "gene_name": "Resistin-like beta",
  "gene_symbol": "RETNLB",
  "gene": "UniProtKB:Q9BQ08",
  "term_id": "UNKNOWN:0001",
  "term_label": "Unknown molecular function"
}